meiotic strand invasion [GO:0000708] (biological process) Definition: The cell cycle process in which the nucleoprotein complex (composed of the broken single-strand DNA and the recombinase) searches and identifies a region of homology in intact duplex DNA. The broken single-strand DNA displaces the like strand and forms Watson-Crick base pairs with its complement, forming a duplex in which each strand is from one of the two recombining DNA molecules. This occurs during meiosis. Also known as: meiotic D-loop biosynthesis, meiotic D-loop formation, meiotic displacement loop biosynthesis, meiotic displacement loop formation Relationships: is a type of DNA strand invasion [GO:0042148]; is a type of GO:0061982 References: PMID:10915877 Sources: GOC:elh Subtypes: GO:0010774, meiotic strand invasion involved in meiotic gene conversion [GO:0010775]